symbiont-mediated induction of syncytium formation [GO:0060141] (biological process) Also known as: positive regulation of syncytium formation by virus, syncytium formation induced by viral infection Sources: GOC:dph Definition: A process in which a symbiont initiates, promotes, or enhances the formation of a syncytium, a mass of cytoplasm containing several nuclei enclosed within a single plasma membrane, by the fusion of the plasma membranes of two or more individual host cells. Syncytia are produced by viruses that are able to fuse directly at the cell surface without requiring endocytosis. Relationships: is a type of GO:0044068